aerobic ammonia oxidation to nitrite via pyruvic oxime [GO:0070275] (biological process) Sources: MetaCyc:PWY-2242 Relationships: is a type of GO:0019329 Definition: The metabolic process in which ammonia (NH3) is oxidized to nitrite (NO2) in the presence of oxygen. Hydroxylamine is produced enzymatically, and, in the presence of pyruvate, forms pyruvic oxime in a spontaneous, non-enzymatic reaction; pyruvic oxime is then converted to nitrite.